{
  "term_id": "GO:0005797",
  "term_label": "Golgi medial cisterna",
  "gene_symbol": "HID1",
  "gene_name": "Protein HID1",
  "gene": "UniProtKB:Q8IV36"
}